positive regulation of vulval development [GO:0040026] (biological process) Also known as: activation of vulval development, stimulation of vulval development, up regulation of vulval development, up-regulation of vulval development, upregulation of vulval development Relationships: is a type of regulation of vulval development [GO:0040028]; is_a GO:0051094; positively regulates vulval development [GO:0040025] Sources: GOC:ems, GOC:kmv Definition: Any process that activates or increases the frequency, rate or extent of development of the vulva. Vulval development is the process whose specific outcome is the progression of the egg-laying organ of female and hermaphrodite nematodes over time, from its formation to the mature structure. In nematodes, the vulva is formed from ventral epidermal cells during larval stages to give rise to a fully formed vulva in the adult.